pyloric antrum smooth muscle contraction [GO:0120065] (biological process) Regulation: regulated by regulation of pyloric antrum smooth muscle contraction [GO:0120071]; positively regulated by GO:0120072; negatively regulated by negative regulation of pyloric antrum smooth muscle contraction [GO:0120073] Also known as: antrum smooth muscle contraction Relationships: is a type of stomach pylorus smooth muscle contraction [GO:0120064] Definition: A process in which force is generated within gastric smooth muscle tissue, resulting in a change in muscle geometry. This process occurs in the widest part of the pylorus that is continuous with the body of the stomach. References: PMID:15890336 Sources: GOC:sl